{
  "gene_symbol": "PKD2",
  "term_label": "membrane",
  "gene_name": "Polycystin-2",
  "term_id": "GO:0016020",
  "gene": "UniProtKB:Q13563"
}